{
  "gene_symbol": "JSRP1",
  "gene": "UniProtKB:Q96MG2",
  "gene_name": "Junctional sarcoplasmic reticulum protein 1",
  "term_label": "Unknown molecular function",
  "term_id": "UNKNOWN:0001"
}